{
  "gene_name": "Ketosamine-3-kinase",
  "gene_symbol": "FN3KRP",
  "term_id": "UNKNOWN:0003",
  "term_label": "Unknown cellular component",
  "gene": "UniProtKB:Q9HA64"
}